{
  "gene_symbol": "FAM107B",
  "term_label": "Unknown molecular function",
  "gene": "UniProtKB:Q9H098",
  "term_id": "UNKNOWN:0001",
  "gene_name": "Protein FAM107B"
}